{
  "term_id": "GO:0005783",
  "term_label": "endoplasmic reticulum",
  "gene_name": "Prolyl 4-hydroxylase subunit alpha-1",
  "gene_symbol": "P4HA1",
  "gene": "UniProtKB:P13674"
}